{
  "gene": "UniProtKB:Q06187",
  "gene_symbol": "BTK",
  "term_id": "GO:0004715",
  "gene_name": "Tyrosine-protein kinase BTK",
  "term_label": "non-membrane spanning protein tyrosine kinase activity"
}